{
  "gene_symbol": "CACNA2D3",
  "gene_name": "Voltage-dependent calcium channel subunit alpha-2_delta-3",
  "term_label": "voltage-gated calcium channel complex",
  "term_id": "GO:0005891",
  "gene": "UniProtKB:Q8IZS8"
}